{
  "term_id": "UNKNOWN:0001",
  "gene": "UniProtKB:Q96FA7",
  "term_label": "Unknown molecular function",
  "gene_name": "Putative protein ZBED10P",
  "gene_symbol": "ZBED10P"
}